regulation of muscle contraction [GO:0006937] (biological process) Sources: GOC:go_curators Subtypes: GO:0006940, GO:0006942, regulation of muscle filament sliding [GO:0032971], negative regulation of muscle contraction [GO:0045932], positive regulation of muscle contraction [GO:0045933] Relationships: is a type of regulation of muscle system process [GO:0090257]; regulates GO:0006936 Definition: Any process that modulates the frequency, rate or extent of muscle contraction.